thiamine oxidase activity [GO:0050423] (molecular function) Sources: EC:1.1.3.23, MetaCyc:THIAMIN-OXIDASE-RXN Relationships: is_a oxidoreductase activity, acting on the CH-OH group of donors, oxygen as acceptor [GO:0016899] Definition: Catalysis of the reaction: thiamine + 2 O2 = thiamine acetic acid + 2 H2O2. Also known as: thiamin oxidase activity, thiamin dehydrogenase activity, thiamin:oxygen 5-oxidoreductase activity, thiamine dehydrogenase activity, thiamine:oxygen 5-oxidoreductase activity